{
  "term_id": "GO:0031146",
  "gene": "UniProtKB:Q93034",
  "gene_symbol": "CUL5",
  "gene_name": "Cullin-5",
  "term_label": "SCF-dependent proteasomal ubiquitin-dependent protein catabolic process"
}